{
  "term_id": "GO:0005737",
  "gene_name": "FH1_FH2 domain-containing protein 1",
  "gene": "UniProtKB:Q9Y613",
  "gene_symbol": "FHOD1",
  "term_label": "cytoplasm"
}